{
  "gene_name": "Kinesin-associated protein 3",
  "gene_symbol": "KIFAP3",
  "gene": "UniProtKB:Q92845",
  "term_label": "kinesin II complex",
  "term_id": "GO:0016939"
}